regulation of systemic arterial blood pressure by epinephrine [GO:0003047] (biological process) Definition: The regulation of blood pressure mediated by the catecholamine signaling molecule epinephrine. Sources: GOC:mtg_cardio Also known as: regulation of blood pressure by adrenaline, blood pressure regulation by epinephrine Relationships: is a type of regulation of systemic arterial blood pressure mediated by a chemical signal [GO:0003044]; is part of regulation of systemic arterial blood pressure by norepinephrine-epinephrine [GO:0001993]